deoxyadenosine kinase activity [GO:0004136] (molecular function) Sources: EC:2.7.1.76, RHEA:23452 Relationships: is a type of deoxynucleoside kinase activity [GO:0019136]; is part of dAMP biosynthetic process [GO:0006170] Definition: Catalysis of the reaction: 2'-deoxyadenosine + ATP = ADP + dAMP + 2 H+. Also known as: ATP:deoxyadenosine 5'-phosphotransferase activity, deoxyadenosine kinase (phosphorylating), purine-deoxyribonucleoside kinase activity